{
  "gene_symbol": "CARMIL1",
  "term_label": "plasma membrane",
  "term_id": "GO:0005886",
  "gene_name": "F-actin-uncapping protein LRRC16A",
  "gene": "UniProtKB:Q5VZK9"
}